positive regulation of G1 to G0 transition [GO:1903452] (biological process) References: PMID:24088570 Sources: GOC:TermGenie, GOC:di, GO_REF:0000058 Definition: Any process that activates or increases the frequency, rate or extent of G1 to G0 transition. Relationships: is a type of positive regulation of cell cycle process [GO:0090068]; is a type of GO:1903450; positively regulates G1 to G0 transition [GO:0070314] Also known as: positive regulation of G1/G0 transition, positive regulation of establishment of cell quiescence, up regulation of G1 to G0 transition, up regulation of G1/G0 transition, up regulation of establishment of cell quiescence, up-regulation of G1 to G0 transition, up-regulation of G1/G0 transition, up-regulation of establishment of cell quiescence, upregulation of G1 to G0 transition, upregulation of G1/G0 transition, upregulation of establishment of cell quiescence, activation of G1 to G0 transition, activation of G1/G0 transition, activation of establishment of cell quiescence, activation of cell cycle quiescence, activation of stationary phase, positive regulation of cell cycle quiescence, positive regulation of stationary phase, up regulation of cell cycle quiescence, up regulation of stationary phase, up-regulation of cell cycle quiescence, up-regulation of stationary phase, upregulation of cell cycle quiescence, upregulation of stationary phase